{
  "term_label": "endoderm formation",
  "gene_name": "Dual specificity protein phosphatase 1",
  "gene_symbol": "DUSP1",
  "gene": "UniProtKB:P28562",
  "term_id": "GO:0001706"
}